{
  "gene_symbol": "PGPEP1",
  "term_id": "GO:0008233",
  "term_label": "peptidase activity",
  "gene_name": "Pyroglutamyl-peptidase 1",
  "gene": "UniProtKB:Q9NXJ5"
}